trigeminal motor nucleus development [GO:0021731] (BP) Relationships: is a type of GO:0048857; is part of pons development [GO:0021548] Definition: The process whose specific outcome is the progression of the trigeminal motor nucleus over time, from its formation to the mature structure. Sources: GOC:cls, GOC:curators, GOC:dgh, GOC:dph, GOC:jid